{
  "term_label": "DNA damage response",
  "gene": "UniProtKB:P22314",
  "gene_symbol": "UBA1",
  "term_id": "GO:0006974",
  "gene_name": "Ubiquitin-like modifier-activating enzyme 1"
}